{
  "gene_name": "HLA class II histocompatibility antigen, DM beta chain",
  "term_label": "peptide antigen binding",
  "term_id": "GO:0042605",
  "gene": "UniProtKB:P28068",
  "gene_symbol": "HLA-DMB"
}